{
  "term_label": "cellular response to oxidative stress",
  "term_id": "GO:0034599",
  "gene_name": "Glutathione peroxidase 3",
  "gene_symbol": "GPX3",
  "gene": "UniProtKB:P22352"
}